{
  "gene_name": "Thromboxane A2 receptor",
  "gene_symbol": "TBXA2R",
  "gene": "UniProtKB:P21731",
  "term_id": "GO:0007189",
  "term_label": "adenylate cyclase-activating G protein-coupled receptor signaling pathway"
}